positive regulation of amyloid precursor protein biosynthetic process [GO:0042986] (BP) Also known as: positive regulation of APP biosynthesis, positive regulation of APP biosynthetic process, positive regulation of amyloid precursor protein anabolism, positive regulation of amyloid precursor protein biosynthesis, positive regulation of amyloid precursor protein formation, positive regulation of amyloid precursor protein synthesis, up regulation of amyloid precursor protein biosynthetic process, up-regulation of amyloid precursor protein biosynthetic process, upregulation of amyloid precursor protein biosynthetic process, activation of amyloid precursor protein biosynthetic process, stimulation of amyloid precursor protein biosynthetic process Sources: GOC:go_curators Relationships: is a type of positive regulation of glycoprotein biosynthetic process [GO:0010560]; is a type of regulation of amyloid precursor protein biosynthetic process [GO:0042984]; positively regulates GO:0042983 Definition: Any process that activates or increases the frequency, rate or extent of the chemical reactions and pathways resulting in the formation of amyloid precursor protein (APP), the precursor of amyloid-beta.